{
  "gene_symbol": "OR14I1",
  "term_id": "UNKNOWN:0003",
  "gene_name": "Olfactory receptor 14I1",
  "term_label": "Unknown cellular component",
  "gene": "UniProtKB:A6ND48"
}